chromocenter [GO:0010369] (cellular component) Subtypes: polytene chromosome chromocenter [GO:0005701], perinucleolar chromocenter [GO:0010370] Definition: A region in which centric, heterochromatic portions from more than one chromosomes form a compact structure. Relationships: is a type of intracellular membraneless organelle [GO:0043232] References: PMID:12384572, PMID:15053486, PMID:16831888